tRNA modification guide activity [GO:0030557] (molecular function) Note: Note that this term describes the activity of a nucleic acid, usually RNA, gene product that interacts with other RNA molecules via base pairing; it should not be used to annotate proteins. Definition: Specifies the site of a posttranscriptional modification in a tRNA molecule by base pairing with a short sequence around the target residue. Subtypes: tRNA pseudouridylation guide activity [GO:0030560], tRNA 2'-O-ribose methylation guide activity [GO:0030564] Relationships: is a type of tRNA binding [GO:0000049]; is a type of RNA modification guide activity [GO:0030555] References: PMID:12457565 Sources: GOC:mah